negative regulation of response to water deprivation [GO:0080148] (biological process) Definition: Any process that stops, prevents, or reduces the frequency, rate or extent of a response to water deprivation. Response to water deprivation is a change in state or activity of a cell or an organism (in terms of movement, secretion, enzyme production, gene expression, etc.) as a result of a water deprivation stimulus, prolonged deprivation of water. References: PMID:18835996 Relationships: is a type of GO:0048585; is a type of GO:2000070; RO_0002212 response to water deprivation [GO:0009414]